{
  "gene_name": "T-cell antigen CD7",
  "term_id": "UNKNOWN:0001",
  "gene_symbol": "CD7",
  "term_label": "Unknown molecular function",
  "gene": "UniProtKB:P09564"
}